oxidoreductase activity, acting on peroxide as acceptor [GO:0016684] (molecular function) Definition: Catalysis of an oxidation-reduction (redox) reaction in which the peroxide group acts as a hydrogen or electron acceptor. Subtypes: peroxidase activity [GO:0004601], GO:1990137 Sources: EC:1.11.-.- Relationships: is a type of oxidoreductase activity [GO:0016491]